somite development [GO:0061053] (biological process) Definition: The progression of a somite from its initial formation to the mature structure. Somites are mesodermal clusters that are arranged segmentally along the anterior posterior axis of an embryo. Sources: GOC:dph Relationships: is a type of epithelium development [GO:0060429]; is part of GO:0009790